endodermal cell fate determination [GO:0007493] (biological process) Also known as: endoderm cell fate determination Relationships: is a type of GO:0001709; is part of GO:0001711 Note: Note that this term was 'endoderm determination'. Changed string to make it more consistent with parent term 'cell fate determination'. Definition: The cell fate determination process in which a cell becomes capable of differentiating autonomously into an endoderm cell regardless of its environment; upon determination, the cell fate cannot be reversed. Sources: GOC:go_curators, ISBN:0878932437